protocadherin-alpha-v4-protocadherin-gamma-b2 complex [GO:0071186] (CC) Also known as: Pcdhga1-Pcdhgb2 complex Definition: A protein complex that contains the cell adhesion molecules protocadherin-alpha-v4 and protocadherin-gamma-b2, and is involved in the regulation of protein localization to the plasma membrane. Relationships: is a type of protocadherin-alpha-protocadherin-gamma complex [GO:0071183] References: PMID:15347688